peroxisome targeting sequence binding [GO:0000268] (molecular function) Definition: Binding to a peroxisomal targeting sequence, a sequence of amino acids within a protein that acts as a signal for the localization of a protein into the peroxisome. Sources: GOC:mah, ISBN:0879693568 Also known as: PTS binding, PTS receptor, peroxisome targeting signal receptor Relationships: is a type of signal sequence binding [GO:0005048] Subtypes: peroxisome matrix targeting signal-1 binding [GO:0005052], peroxisome matrix targeting signal-2 binding [GO:0005053], peroxisome membrane targeting sequence binding [GO:0033328]